peptidyl-histidine dioxygenase activity [GO:0036139] (MF) Definition: Catalysis of the reaction: L-histidyl-[protein] + 2-oxoglutarate + O2 = (3S)-3-hydroxy-L-histidyl-[protein] + succinate + CO2. References: PMID:21251231 Sources: RHEA:54256 Also known as: protein histidyl hydroxylase, protein-L-histidine (3S)-3-hydroxylase Relationships: is a type of GO:0016706; is a type of catalytic activity, acting on a protein [GO:0140096]